{
  "gene_name": "Uncharacterized protein C20orf96",
  "gene_symbol": "C20orf96",
  "term_id": "UNKNOWN:0002",
  "gene": "UniProtKB:Q9NUD7",
  "term_label": "Unknown biological process"
}